{
  "gene": "UniProtKB:Q96PP9",
  "term_label": "defense response to Gram-positive bacterium",
  "gene_symbol": "GBP4",
  "term_id": "GO:0050830",
  "gene_name": "Guanylate-binding protein 4"
}